{
  "gene_name": "Histone RNA hairpin-binding protein",
  "term_label": "mRNA transport",
  "term_id": "GO:0051028",
  "gene_symbol": "SLBP",
  "gene": "UniProtKB:Q14493"
}